{
  "gene": "UniProtKB:O43379",
  "term_label": "spindle pole",
  "gene_symbol": "WDR62",
  "gene_name": "WD repeat-containing protein 62",
  "term_id": "GO:0000922"
}